{
  "gene_name": "Zinc finger protein 79",
  "term_id": "GO:0000981",
  "term_label": "DNA-binding transcription factor activity, RNA polymerase II-specific",
  "gene_symbol": "ZNF79",
  "gene": "UniProtKB:Q15937"
}